{
  "gene_symbol": "NDUFS1",
  "gene": "UniProtKB:P28331",
  "term_label": "mitochondrial respiratory chain complex I assembly",
  "term_id": "GO:0032981",
  "gene_name": "NADH-ubiquinone oxidoreductase 75 kDa subunit, mitochondrial"
}